beta-L-rhamnosidase activity [GO:0033908] (MF) Sources: EC:3.2.1.43 Relationships: is a type of hydrolase activity, hydrolyzing O-glycosyl compounds [GO:0004553] Definition: Catalysis of the hydrolysis of terminal, non-reducing beta-L-rhamnose residues in beta-L-rhamnosides. Also known as: beta-L-rhamnoside rhamnohydrolase activity